{
  "gene_symbol": "ARHGEF16",
  "gene": "UniProtKB:Q5VV41",
  "gene_name": "Rho guanine nucleotide exchange factor 16",
  "term_label": "regulation of Cdc42 protein signal transduction",
  "term_id": "GO:0032489"
}